{
  "gene_name": "Putative BPES syndrome breakpoint region protein",
  "term_label": "Unknown biological process",
  "gene_symbol": "BPESC1",
  "gene": "UniProtKB:Q9GZL8",
  "term_id": "UNKNOWN:0002"
}